forebrain cell migration [GO:0021885] (biological process) Definition: The orderly movement of a cell from one site to another at least one of which is located in the forebrain. Relationships: is a type of GO:0016477; BFO_0000050 forebrain development [GO:0030900] Subtypes: GO:0022029, GO:0061381 Sources: GOC:cls, GOC:dgh, GOC:dph, GOC:jid, GO_REF:0000021